double stranded viral RNA replication [GO:0039691] (biological process) Sources: GOC:bf, GOC:jl, VZ:1936 Definition: A viral genome replication process where the template genome is double stranded RNA (dsRNA). Genomic dsRNA is first transcribed into single-stranded (ss) mRNA, which is then replicated to ds-genomic RNA. Relationships: is a type of GO:0039694; has part RNA-templated viral transcription [GO:0039696]